{
  "term_label": "Unknown molecular function",
  "gene_symbol": "CASC2",
  "term_id": "UNKNOWN:0001",
  "gene_name": "Protein CASC2, isoform 3",
  "gene": "UniProtKB:Q6XLA1"
}